{
  "gene_name": "Poly(rC)-binding protein 1",
  "gene_symbol": "PCBP1",
  "term_id": "GO:0005634",
  "gene": "UniProtKB:Q15365",
  "term_label": "nucleus"
}